maltoheptaose binding [GO:2001071] (molecular function) Relationships: is a type of GO:0070492 Sources: GOC:mengo_curators Definition: Binding to maltoheptaose.